host interaction involved in quorum sensing [GO:0120218] (biological process) Relationships: is a type of quorum sensing [GO:0009372] References: PMID:11780122, PMID:16630813 Sources: GOC:krc, GOC:mlg Definition: A quorum sensing process that is modulated by some interaction with a host cell or organism.